neuronal action potential propagation [GO:0019227] (biological process) Definition: The propagation of an action potential along an axon, away from the soma. Sources: GOC:isa_complete Relationships: is a type of nervous system process [GO:0050877]; is a type of action potential propagation [GO:0098870]; is part of transmission of nerve impulse [GO:0019226]